{
  "term_label": "amyloid-beta metabolic process",
  "term_id": "GO:0050435",
  "gene_symbol": "BACE1",
  "gene_name": "Beta-secretase 1",
  "gene": "UniProtKB:P56817"
}